{
  "gene_name": "Olfactory receptor 7G3",
  "term_id": "GO:0004984",
  "gene_symbol": "OR7G3",
  "gene": "UniProtKB:Q8NG95",
  "term_label": "olfactory receptor activity"
}